growth factor receptor binding [GO:0070851] (molecular function) Sources: GOC:mah, GOC:vw Definition: Binding to a growth factor receptor. Subtypes: fibroblast growth factor receptor binding [GO:0005104], granulocyte macrophage colony-stimulating factor receptor binding [GO:0005129], granulocyte colony-stimulating factor receptor binding [GO:0005130], GO:0005134, interleukin-3 receptor binding [GO:0005135], interleukin-4 receptor binding [GO:0005136], interleukin-5 receptor binding [GO:0005137], interleukin-6 receptor binding [GO:0005138], GO:0005139, GO:0005140, interleukin-10 receptor binding [GO:0005141], interleukin-11 receptor binding [GO:0005142], GO:0005143, interleukin-1 receptor binding [GO:0005149], epidermal growth factor receptor binding [GO:0005154], GO:0005161, GO:0005171, vascular endothelial growth factor receptor binding [GO:0005172], imaginal disc growth factor receptor binding [GO:0008084], glial cell-derived neurotrophic factor receptor binding [GO:0030116], GO:0030372 Relationships: is a type of GO:0005102